{
  "gene_name": "Homeobox protein Nkx-2.3",
  "term_id": "GO:0000981",
  "gene_symbol": "NKX2-3",
  "gene": "UniProtKB:Q8TAU0",
  "term_label": "DNA-binding transcription factor activity, RNA polymerase II-specific"
}